positive regulation of glutamatergic neuron differentiation [GO:0120008] (biological process) Definition: Any process that activates or increases the frequency, rate or extent of glutamatergic neuron differentiation. Relationships: is a type of positive regulation of neuron differentiation [GO:0045666]; is a type of regulation of glutamatergic neuron differentiation [GO:0120006]; positively regulates GO:1905962 References: PMID:24030726